positive regulation of T-helper 1 cell activation [GO:2000519] (biological process) Definition: Any process that activates or increases the frequency, rate or extent of T-helper 1 cell activation. Sources: GOC:obol Also known as: positive regulation of Th1 cell activation Relationships: is_a positive regulation of CD4-positive, alpha-beta T cell activation [GO:2000516]; is a type of GO:2000517; positively regulates T-helper 1 cell activation [GO:0035711]